{
  "term_id": "GO:0006357",
  "gene": "UniProtKB:Q96QS3",
  "gene_name": "Homeobox protein ARX",
  "term_label": "regulation of transcription by RNA polymerase II",
  "gene_symbol": "ARX"
}